DNA demethylase activity [GO:0035514] (MF) Relationships: is a type of demethylase activity [GO:0032451]; is a type of catalytic activity, acting on DNA [GO:0140097] Definition: Catalysis of the removal of a methyl group from one or more nucleosides within a DNA molecule. Subtypes: broad specificity oxidative DNA demethylase activity [GO:0035516], cytosine C-5 DNA demethylase activity [GO:0051747], DNA N6-methyladenine demethylase activity [GO:0141131] Sources: GOC:bf